positive regulation of immune response to tumor cell [GO:0002839] (biological process) Subtypes: positive regulation of T cell mediated immune response to tumor cell [GO:0002842], positive regulation of tolerance induction to tumor cell [GO:0002845], positive regulation of natural killer cell mediated immune response to tumor cell [GO:0002857] Relationships: is a type of positive regulation of response to tumor cell [GO:0002836]; is a type of GO:0002837; is a type of positive regulation of immune response [GO:0050778]; positively regulates immune response to tumor cell [GO:0002418] Also known as: positive regulation of immune response to tumour cell, up regulation of immune response to tumor cell, up-regulation of immune response to tumor cell, upregulation of immune response to tumor cell, activation of immune response to tumor cell, stimulation of immune response to tumor cell Definition: Any process that activates or increases the frequency, rate, or extent of an immune response to tumor cell. Sources: GOC:add